{
  "gene_symbol": "KLHDC1",
  "term_id": "UNKNOWN:0001",
  "gene": "UniProtKB:Q8N7A1",
  "term_label": "Unknown molecular function",
  "gene_name": "Kelch domain-containing protein 1"
}